{
  "gene": "UniProtKB:Q8WV41",
  "gene_name": "Sorting nexin-33",
  "gene_symbol": "SNX33",
  "term_id": "GO:0005886",
  "term_label": "plasma membrane"
}